{
  "gene_name": "CDK5 and ABL1 enzyme substrate 1",
  "gene_symbol": "CABLES1",
  "term_label": "cytosol",
  "gene": "UniProtKB:Q8TDN4",
  "term_id": "GO:0005829"
}